non-professional antigen presenting cell antigen processing and presentation [GO:0002473] (biological process) Relationships: is a type of GO:0019882 Definition: The process in which a non-professional antigen presenting cell expresses antigen (peptide or lipid) on its cell surface in association with an MHC protein complex. Non-professional antigen presenting cells include all cell types but dendritic cells, B cells, T cells, monocytes, macrophages, and neutrophils. Regulation: regulated by regulation of non-professional antigen presenting cell antigen processing and presentation [GO:0002619]; RO_0002212 by negative regulation of non-professional antigen presenting cell antigen processing and presentation [GO:0002620]; RO_0002213 by positive regulation of non-professional antigen presenting cell antigen processing and presentation [GO:0002621] References: PMID:15771591 Sources: GOC:add, ISBN:0781735149